putrescine N-hydroxycinnamoyltransferase activity [GO:0047174] (molecular function) Relationships: is a type of N-acyltransferase activity [GO:0016410]; is a type of GO:0050734 Definition: Catalysis of the reaction: caffeoyl-CoA + putrescine = N-caffeoylputrescine + CoA + H+. Also known as: PHT, caffeoyl-CoA putrescine N-caffeoyl transferase activity, caffeoyl-CoA:putrescine N-(3,4-dihydroxycinnamoyl)transferase activity, hydroxycinnamoyl-CoA:putrescine hydroxycinnamoyltransferase activity, putrescine hydroxycinnamoyl transferase activity, putrescine hydroxycinnamoyltransferase activity Sources: EC:2.3.1.138, RHEA:12436